regulation of methane biosynthetic process from methylamine [GO:1900348] (biological process) Relationships: is a type of regulation of amine metabolic process [GO:0033238]; is a type of regulation of cellular respiration [GO:0043457]; is a type of regulation of alkane biosynthetic process [GO:1901577]; RO_0002211 methane biosynthetic process from methylamine [GO:2001128] Subtypes: negative regulation of methane biosynthetic process from methylamine [GO:1900349], GO:1900350 Sources: GOC:TermGenie, GOC:mengo_curators Definition: Any process that modulates the frequency, rate or extent of methane biosynthetic process from methylamine.